{
  "gene_symbol": "TSPYL4",
  "gene": "UniProtKB:Q9UJ04",
  "term_label": "histone binding",
  "term_id": "GO:0042393",
  "gene_name": "Testis-specific Y-encoded-like protein 4"
}